{
  "gene_name": "E3 ubiquitin-protein ligase UBR3",
  "term_id": "GO:0005737",
  "gene_symbol": "UBR3",
  "term_label": "cytoplasm",
  "gene": "UniProtKB:Q6ZT12"
}